{
  "term_id": "GO:0005813",
  "gene_name": "Rootletin",
  "gene_symbol": "CROCC",
  "gene": "UniProtKB:Q5TZA2",
  "term_label": "centrosome"
}